{
  "gene_name": "Neuronal acetylcholine receptor subunit alpha-6",
  "term_label": "acetylcholine-gated monoatomic cation-selective channel activity",
  "gene_symbol": "CHRNA6",
  "gene": "UniProtKB:Q15825",
  "term_id": "GO:0022848"
}